phloem nitrate loading [GO:0090408] (biological process) Relationships: is a type of GO:0015706; is a type of phloem loading [GO:0110126] Definition: The process of loading nitrate into the sieve tube or companion cell of the phloem for long distance transport from source to sink. Sources: GOC:tb